{
  "gene_name": "2-oxoglutarate and iron-dependent oxygenase domain-containing protein 2",
  "gene": "UniProtKB:Q6N063",
  "term_id": "UNKNOWN:0002",
  "term_label": "Unknown biological process",
  "gene_symbol": "OGFOD2"
}